{
  "term_label": "Unknown cellular component",
  "term_id": "UNKNOWN:0003",
  "gene_symbol": "NXPH3",
  "gene": "UniProtKB:O95157",
  "gene_name": "Neurexophilin-3"
}